{
  "gene_name": "Potassium voltage-gated channel subfamily D member 3",
  "gene": "UniProtKB:Q9UK17",
  "gene_symbol": "KCND3",
  "term_id": "GO:0008076",
  "term_label": "voltage-gated potassium channel complex"
}